{
  "gene_symbol": "TMEM88",
  "term_label": "Unknown molecular function",
  "gene": "UniProtKB:Q6PEY1",
  "gene_name": "Transmembrane protein 88",
  "term_id": "UNKNOWN:0001"
}